{
  "term_id": "UNKNOWN:0001",
  "gene": "UniProtKB:Q6ZQY2",
  "term_label": "Unknown molecular function",
  "gene_name": "Leucine-rich repeat-containing protein 74B",
  "gene_symbol": "LRRC74B"
}